{
  "term_id": "GO:0030425",
  "gene_name": "Muscarinic acetylcholine receptor M3",
  "term_label": "dendrite",
  "gene": "UniProtKB:P20309",
  "gene_symbol": "CHRM3"
}